{
  "gene_name": "Calcium-transporting ATPase type 2C member 1",
  "gene": "UniProtKB:P98194",
  "gene_symbol": "ATP2C1",
  "term_id": "GO:0006874",
  "term_label": "intracellular calcium ion homeostasis"
}